{
  "gene_symbol": "B4GALNT2",
  "term_id": "GO:0008376",
  "gene_name": "Beta-1,4 N-acetylgalactosaminyltransferase 2",
  "gene": "UniProtKB:Q8NHY0",
  "term_label": "acetylgalactosaminyltransferase activity"
}